negative regulation of lipase activity [GO:0060192] (biological process) Relationships: is a type of negative regulation of hydrolase activity [GO:0051346]; negatively regulates lipase activity [GO:0016298] Subtypes: negative regulation of lipoprotein lipase activity [GO:0051005] Sources: GOC:dph, GOC:tb Definition: Any process that decreases the frequency, rate or extent of lipase activity, the hydrolysis of a lipid or phospholipid.